{
  "term_id": "GO:0005332",
  "gene": "UniProtKB:P48029",
  "term_label": "gamma-aminobutyric acid:sodium:chloride symporter activity",
  "gene_symbol": "SLC6A8",
  "gene_name": "Sodium- and chloride-dependent creatine transporter 1"
}